{
  "gene_symbol": "CAND1",
  "gene": "UniProtKB:Q86VP6",
  "gene_name": "Cullin-associated NEDD8-dissociated protein 1",
  "term_id": "GO:0005634",
  "term_label": "nucleus"
}